{
  "gene": "UniProtKB:Q15784",
  "gene_symbol": "NEUROD2",
  "term_label": "positive regulation of transcription by RNA polymerase II",
  "gene_name": "Neurogenic differentiation factor 2",
  "term_id": "GO:0045944"
}